NK T cell lineage commitment [GO:0002364] (BP) Definition: The process in which a pro-T cell becomes committed to becoming an NK T cell. Sources: GOC:add, ISBN:0781735149 Also known as: NK T lymphocyte lineage commitment, NK T-cell lineage commitment, NK T-lymphocyte lineage commitment, natural killer T lymphocyte lineage commitment, natural killer T-cell lineage commitment, natural killer T-lymphocyte lineage commitment Relationships: is a type of GO:0002363; is part of GO:0001865